{
  "term_id": "GO:0002151",
  "term_label": "G-quadruplex RNA binding",
  "gene_symbol": "DHX30",
  "gene": "UniProtKB:Q7L2E3",
  "gene_name": "ATP-dependent RNA helicase DHX30"
}